regulation of optic nerve formation [GO:2000595] (biological process) Definition: Any process that modulates the frequency, rate or extent of optic nerve formation. Sources: GOC:obol Subtypes: negative regulation of optic nerve formation [GO:2000596], positive regulation of optic nerve formation [GO:2000597] Relationships: is_a regulation of anatomical structure morphogenesis [GO:0022603]; regulates optic nerve formation [GO:0021634] Also known as: regulation of CN II biosynthesis, regulation of CN II formation